{
  "gene": "UniProtKB:P01344",
  "term_label": "extracellular space",
  "gene_symbol": "IGF2",
  "term_id": "GO:0005615",
  "gene_name": "Insulin-like growth factor II"
}